negative regulation of seed maturation [GO:2000692] (biological process) Definition: Any process that stops, prevents or reduces the frequency, rate or extent of seed maturation. Sources: GOC:obol Relationships: is_a negative regulation of developmental process [GO:0051093]; is a type of negative regulation of multicellular organismal process [GO:0051241]; is a type of GO:2000034; is a type of GO:2000242; negatively regulates seed maturation [GO:0010431]